vacuolar lumen [GO:0005775] (cellular component) Sources: ISBN:0198506732 Subtypes: fungal-type vacuole lumen [GO:0000328], plant-type vacuole lumen [GO:0000330], autophagosome lumen [GO:0034423], azurophil granule lumen [GO:0035578], GO:0043202, phagolysosome vesicle lumen [GO:0106174], autolysosome lumen [GO:0120282], GO:1904856 Definition: The volume enclosed within the vacuolar membrane. Relationships: is a type of GO:0070013; is part of GO:0005773